ribonuclease T2 activity [GO:0033897] (molecular function) Also known as: RNase II activity, ribonuclease II activity, ribonucleate nucleotido-2'-transferase (cyclizing) activity, Escherichia coli ribonuclease I' ribonuclease PP2 activity, RNAase CL activity, RNase (non-base specific) activity, RNase Ms activity, acid RNase activity, acid ribonuclease activity, base-non-specific ribonuclease activity, non-base specific ribonuclease activity, nonbase-specific RNase activity, nonspecific RNase activity, ribonnuclease (non-base specific) activity, ribonuclease M activity, ribonuclease N2 activity, ribonuclease U4 activity, ribonucleate 3'-oligonucleotide hydrolase activity, Escherichia coli ribonuclease II activity, RNase M activity, RNase T2 activity, ribonuclease (non-base specific) activity, ribonuclease PP3 activity Sources: EC:4.6.1.19, RHEA:68052 Relationships: is_a GO:0004521; is a type of GO:0016849 Definition: Catalysis of the reaction: a ribonucleotidyl-ribonucleotide-RNA + H2O = a 3'-end 3'-phospho-ribonucleotide-RNA + a 5'-end dephospho-ribonucleoside-RNA + H+. This reaction is a two-stage endonucleolytic cleavage to nucleoside 3'-phosphates and 3'-phosphooligonucleotides with 2',3'-cyclic phosphate intermediates.